epigenetic programing of male pronucleus [GO:0044727] (biological process) Also known as: epigenetic reprograming of male pronucleus, epigenetic reprograming of paternal genome in zygote, DNA demethylation of male pronucleus Definition: The global programming of epigenetic modifications in the male pronucleus of the newly fertilized zygote. The most major change in the paternal genome is DNA demethylation, which takes place before the first cell division. References: PMID:22868271 Sources: GOC:sp Relationships: is a type of GO:0044725